{
  "gene_name": "Histone acetyltransferase KAT7",
  "gene_symbol": "KAT7",
  "term_label": "chromatin binding",
  "gene": "UniProtKB:O95251",
  "term_id": "GO:0003682"
}